{
  "term_label": "chromatin binding",
  "gene_name": "Transcriptional adapter 2-alpha",
  "gene": "UniProtKB:O75478",
  "term_id": "GO:0003682",
  "gene_symbol": "TADA2A"
}